{
  "gene_symbol": "CDK5",
  "gene": "UniProtKB:Q00535",
  "gene_name": "Cyclin-dependent kinase 5",
  "term_id": "GO:1901987",
  "term_label": "regulation of cell cycle phase transition"
}